{
  "term_label": "ubiquitin protein ligase activity",
  "term_id": "GO:0061630",
  "gene_name": "E3 ubiquitin-protein ligase E3D",
  "gene": "UniProtKB:Q7Z6J8",
  "gene_symbol": "UBE3D"
}